dissimilatory sulfite reductase (NADH) activity [GO:0018551] (molecular function) Sources: RHEA:78943 Also known as: siroheme sulfite reductase activity Definition: Catalysis of the reactions: [DsrC protein]-trisulfide + 3 H2O + NAD+ = [DsrC protein]-dithiol + 3 H+ + NADH + sulfite. Relationships: is a type of oxidoreductase activity, acting on a sulfur group of donors, NAD(P) as acceptor [GO:0016668]